{
  "gene": "UniProtKB:A6NEQ2",
  "gene_name": "Protein FAM181B",
  "term_label": "Unknown biological process",
  "term_id": "UNKNOWN:0002",
  "gene_symbol": "FAM181B"
}